aldosterone biosynthetic process [GO:0032342] (biological process) Definition: The chemical reactions and pathways resulting in the formation of aldosterone, a corticosteroid hormone that is produced by the zona glomerulosa of the adrenal cortex and regulates salt (sodium and potassium) and water balance. Regulation: regulated by regulation of aldosterone biosynthetic process [GO:0032347]; negatively regulated by negative regulation of aldosterone biosynthetic process [GO:0032348]; positively regulated by positive regulation of aldosterone biosynthetic process [GO:0032349] Relationships: is a type of C21-steroid hormone biosynthetic process [GO:0006700]; is a type of mineralocorticoid biosynthetic process [GO:0006705]; is a type of GO:0032341; is_a primary alcohol biosynthetic process [GO:0034309]; is a type of GO:0042181; is a type of aldehyde biosynthetic process [GO:0046184]; is a type of olefinic compound biosynthetic process [GO:0120255] References: PMID:16527843